GDP-alpha-D-mannosylchitobiosyldiphosphodolichol biosynthetic process [GO:0019347] (biological process) Definition: The chemical reactions and pathways resulting in the formation of GDP-alpha-D-mannosylchitobiosyldiphosphodolichol, a substance composed of mannosylchitobiosyldiphosphodolichol in glycosidic linkage with guanosine diphosphate. Also known as: GDP-alpha-D-mannosylchitobiosyldiphosphodolichol anabolism, GDP-alpha-D-mannosylchitobiosyldiphosphodolichol biosynthesis, GDP-alpha-D-mannosylchitobiosyldiphosphodolichol formation, GDP-alpha-D-mannosylchitobiosyldiphosphodolichol synthesis Sources: GOC:ai Relationships: is a type of phospholipid biosynthetic process [GO:0008654]; is_a GO:0009247; is a type of terpenoid biosynthetic process [GO:0016114]; is a type of nucleoside phosphate biosynthetic process [GO:1901293]